{
  "gene": "UniProtKB:A0PJX0",
  "gene_name": "Calcium and integrin-binding family member 4",
  "term_id": "UNKNOWN:0002",
  "gene_symbol": "CIB4",
  "term_label": "Unknown biological process"
}